{
  "term_id": "GO:0045177",
  "gene_symbol": "SVBP",
  "gene_name": "Small vasohibin-binding protein",
  "gene": "UniProtKB:Q8N300",
  "term_label": "apical part of cell"
}